{
  "term_label": "choline O-acetyltransferase activity",
  "term_id": "GO:0004102",
  "gene": "UniProtKB:P28329",
  "gene_name": "Choline O-acetyltransferase",
  "gene_symbol": "CHAT"
}